{
  "gene_symbol": "TPSB2",
  "term_label": "proteolysis",
  "gene_name": "Tryptase beta-2",
  "gene": "UniProtKB:P20231",
  "term_id": "GO:0006508"
}